inositol-1,4,5,6-tetrakisphosphate 2-kinase activity [GO:0032942] (molecular function) Definition: Catalysis of the reaction: 1D-myo-inositol 1,4,5,6-tetrakisphosphate + ATP = 1D-myo-inositol 1,2,4,5,6-pentakisphosphate + ADP + H+. Also known as: 1D-myo-inositol-tetrakisphosphate 2-kinase activity, inositol tetrakisphosphate 2-kinase activity, inositol-tetrakisphosphate 2-kinase activity Relationships: is a type of inositol tetrakisphosphate kinase activity [GO:0051765] References: PMID:16107538 Sources: MetaCyc:RXN-7182